{
  "gene_name": "Vascular endothelial growth factor D",
  "term_label": "extracellular space",
  "gene_symbol": "VEGFD",
  "term_id": "GO:0005615",
  "gene": "UniProtKB:O43915"
}